{
  "gene_symbol": "EFCAB9",
  "gene_name": "EF-hand calcium-binding domain-containing protein 9",
  "gene": "UniProtKB:A8MZ26",
  "term_id": "GO:0097228",
  "term_label": "sperm principal piece"
}